{
  "gene_name": "Placenta growth factor",
  "term_id": "GO:0002040",
  "gene": "UniProtKB:P49763",
  "term_label": "sprouting angiogenesis",
  "gene_symbol": "PGF"
}